{
  "gene": "UniProtKB:P09001",
  "gene_name": "Large ribosomal subunit protein uL3m",
  "gene_symbol": "MRPL3",
  "term_id": "GO:0003735",
  "term_label": "structural constituent of ribosome"
}